{
  "gene_symbol": "CUL4B",
  "gene_name": "Cullin-4B",
  "term_id": "GO:0006974",
  "gene": "UniProtKB:Q13620",
  "term_label": "DNA damage response"
}